regulation of mononuclear cell proliferation [GO:0032944] (BP) Definition: Any process that modulates the frequency, rate or extent of mononuclear cell proliferation. Sources: GOC:add Also known as: regulation of PBMC proliferation, regulation of peripheral blood mononuclear cell proliferation Relationships: is a type of GO:0070663; regulates mononuclear cell proliferation [GO:0032943] Subtypes: negative regulation of mononuclear cell proliferation [GO:0032945], positive regulation of mononuclear cell proliferation [GO:0032946], regulation of lymphocyte proliferation [GO:0050670]